{
  "term_id": "GO:0001580",
  "gene_symbol": "RTP2",
  "gene": "UniProtKB:Q5QGT7",
  "gene_name": "Receptor-transporting protein 2",
  "term_label": "detection of chemical stimulus involved in sensory perception of bitter taste"
}